{
  "term_id": "UNKNOWN:0003",
  "gene": "UniProtKB:P0C2Y1",
  "gene_name": "Putative neuroblastoma breakpoint family member 7",
  "gene_symbol": "NBPF7P",
  "term_label": "Unknown cellular component"
}